pseudouridine 5'-phosphatase activity [GO:1990738] (molecular function) Definition: Catalysis of the reaction: pseudouridine 5'-phosphate + H2O = pseudouridine + phosphate. References: PMID:20722631 Sources: EC:3.1.3.96 Relationships: is a type of phosphatase activity [GO:0016791]